{
  "gene_name": "Protein cereblon",
  "gene_symbol": "CRBN",
  "gene": "UniProtKB:Q96SW2",
  "term_id": "GO:0043161",
  "term_label": "proteasome-mediated ubiquitin-dependent protein catabolic process"
}